{
  "term_id": "UNKNOWN:0002",
  "gene_symbol": "TMC3",
  "gene": "UniProtKB:Q7Z5M5",
  "gene_name": "Transmembrane channel-like protein 3",
  "term_label": "Unknown biological process"
}